galacturonate binding [GO:0048032] (molecular function) Definition: Binding to a galacturonate. Galacturonate is the anion of galacturonic acid, the uronic acid formally derived from galactose by oxidation of the hydroxymethylene group at C-6 to a carboxyl group. Relationships: is a type of monocarboxylic acid binding [GO:0033293] Also known as: galacturonic acid binding Sources: GOC:jid